{
  "term_id": "UNKNOWN:0003",
  "gene": "UniProtKB:Q58FG1",
  "gene_name": "Putative heat shock protein HSP 90-alpha A4",
  "gene_symbol": "HSP90AA4P",
  "term_label": "Unknown cellular component"
}